{
  "gene": "UniProtKB:Q99732",
  "gene_symbol": "LITAF",
  "term_id": "GO:0098560",
  "gene_name": "Lipopolysaccharide-induced tumor necrosis factor-alpha factor",
  "term_label": "cytoplasmic side of late endosome membrane"
}